{
  "gene": "UniProtKB:Q15691",
  "gene_name": "Microtubule-associated protein RP_EB family member 1",
  "gene_symbol": "MAPRE1",
  "term_label": "cytoplasmic microtubule",
  "term_id": "GO:0005881"
}